{
  "term_label": "cysteine-type peptidase activity",
  "gene_name": "Cystatin-like 1",
  "gene_symbol": "CSTL1",
  "term_id": "GO:0008234",
  "gene": "UniProtKB:Q9H114"
}